{
  "gene_name": "Coiled-coil domain-containing protein 141",
  "gene": "UniProtKB:Q6ZP82",
  "term_label": "Unknown molecular function",
  "term_id": "UNKNOWN:0001",
  "gene_symbol": "CCDC141"
}